IMP dehydrogenase activity [GO:0003938] (molecular function) Definition: Catalysis of the reaction: inosine 5'-phosphate + NAD+ + H2O = xanthosine 5'-phosphate + NADH + H+. Sources: EC:1.1.1.205 Also known as: IMP oxidoreductase activity, IMP:NAD+ oxidoreductase activity, inosinate dehydrogenase activity, inosine 5'-monophosphate dehydrogenase activity, inosine monophosphate dehydrogenase activity, inosine monophosphate oxidoreductase activity, inosine-5'-phosphate dehydrogenase activity, inosinic acid dehydrogenase activity Relationships: is a type of GO:0016616